{
  "gene": "UniProtKB:O95352",
  "term_label": "phagophore assembly site",
  "gene_symbol": "ATG7",
  "term_id": "GO:0000407",
  "gene_name": "Ubiquitin-like modifier-activating enzyme ATG7"
}